regulation of lipoprotein lipid oxidation [GO:0060587] (biological process) Sources: GOC:BHF, GOC:dph, GOC:tb Definition: Any process that modulates the rate, frequency or extent of lipoprotein lipid oxidation. Lipoprotein lipid oxidation is the modification of a lipoprotein by oxidation of the lipid group. Relationships: is a type of regulation of lipid metabolic process [GO:0019216]; is a type of regulation of lipoprotein oxidation [GO:0034442]; regulates GO:0034439 Subtypes: negative regulation of lipoprotein lipid oxidation [GO:0060588]